positive regulation of dopamine secretion [GO:0033603] (biological process) Sources: GOC:sl Definition: Any process that activates or increases the frequency, rate or extent of the regulated release of dopamine. Also known as: up regulation of dopamine secretion, up-regulation of dopamine secretion, upregulation of dopamine secretion, activation of dopamine secretion, stimulation of dopamine secretion Relationships: is a type of regulation of dopamine secretion [GO:0014059]; is a type of positive regulation of catecholamine secretion [GO:0033605]; positively regulates GO:0014046